positive regulation of L-proline import across plasma membrane [GO:1905737] (biological process) Relationships: is_a positive regulation of proline import across plasma membrane [GO:1902836]; is a type of GO:1905735; positively regulates GO:1904271 Definition: Any process that activates or increases the frequency, rate or extent of L-proline import across plasma membrane. References: PMID:24344203 Sources: GOC:TermGenie, GO_REF:0000058